regulation of mitotic metaphase/anaphase transition [GO:0030071] (biological process) Sources: GOC:mah Subtypes: GO:0045841, positive regulation of mitotic metaphase/anaphase transition [GO:0045842], regulation of mitotic cell cycle spindle assembly checkpoint [GO:0090266] Relationships: is a type of regulation of mitotic cell cycle phase transition [GO:1901990]; is a type of regulation of metaphase/anaphase transition of cell cycle [GO:1902099]; regulates metaphase/anaphase transition of mitotic cell cycle [GO:0007091] Definition: Any process that modulates the frequency, rate or extent of the cell cycle process in which a cell progresses from metaphase to anaphase during mitosis, triggered by the activation of the anaphase promoting complex by Cdc20/Sleepy homolog which results in the degradation of Securin.